{
  "gene_symbol": "GPR21",
  "gene": "UniProtKB:Q99679",
  "term_id": "GO:0004930",
  "gene_name": "Probable G-protein coupled receptor 21",
  "term_label": "G protein-coupled receptor activity"
}